{
  "term_id": "GO:0005886",
  "gene": "UniProtKB:P11465",
  "gene_name": "Pregnancy-specific beta-1-glycoprotein 2",
  "term_label": "plasma membrane",
  "gene_symbol": "PSG2"
}